{
  "gene_name": "DAZ-associated protein 2",
  "gene_symbol": "DAZAP2",
  "gene": "UniProtKB:Q15038",
  "term_id": "UNKNOWN:0003",
  "term_label": "Unknown cellular component"
}